hemoglobin biosynthetic process [GO:0042541] (biological process) Definition: The chemical reactions and pathways resulting in the formation of hemoglobin, an oxygen carrying, conjugated protein containing four heme groups and globin. Sources: GOC:jl Also known as: haemoglobin biosynthesis, haemoglobin biosynthetic process, hemoglobin anabolism, hemoglobin biosynthesis, hemoglobin formation, hemoglobin synthesis Relationships: is a type of macromolecule biosynthetic process [GO:0009059]; is a type of hemoglobin metabolic process [GO:0020027] Regulation: regulated by regulation of hemoglobin biosynthetic process [GO:0046984]; positively regulated by positive regulation of hemoglobin biosynthetic process [GO:0046985]; negatively regulated by negative regulation of hemoglobin biosynthetic process [GO:0046986]